{
  "term_id": "GO:0005886",
  "gene_symbol": "GYPA",
  "term_label": "plasma membrane",
  "gene": "UniProtKB:P02724",
  "gene_name": "Glycophorin-A"
}